{
  "term_label": "immunoglobulin mediated immune response",
  "gene_symbol": "IGLC6",
  "gene": "UniProtKB:P0CF74",
  "gene_name": "Immunoglobulin lambda constant 6",
  "term_id": "GO:0016064"
}